iron-cytochrome-c reductase activity [GO:0047726] (molecular function) Definition: Catalysis of the reaction: ferrocytochrome c + Fe3+ = ferricytochrome c + Fe2+. Sources: EC:1.9.98.1, MetaCyc:IRON--CYTOCHROME-C-REDUCTASE-RXN Also known as: ferrocytochrome-c:Fe3+ oxidoreductase activity, iron-cytochrome c reductase activity Relationships: is a type of GO:0016675